RNA destabilization [GO:0050779] (biological process) Sources: GOC:ai Subtypes: GO:0036417, GO:0061157 Definition: Any process that decreases the stability of an RNA molecule, making it more vulnerable to degradative processes. Relationships: is a type of positive regulation of catabolic process [GO:0009896]; is a type of regulation of RNA stability [GO:0043487]; is a type of positive regulation of RNA metabolic process [GO:0051254]; positively regulates RNA catabolic process [GO:0006401]